{
  "gene_name": "Cytoskeleton-associated protein 5",
  "term_label": "microtubule polymerization",
  "gene_symbol": "CKAP5",
  "term_id": "GO:0046785",
  "gene": "UniProtKB:Q14008"
}